choloyl-CoA hydrolase activity [GO:0033882] (MF) Definition: Catalysis of the reaction: choloyl-CoA + H2O = cholate + CoA. Relationships: is a type of GO:0016289 Also known as: peroxisomal acyl-CoA thioesterase 2 activity, PTE-2, chenodeoxycholoyl-coenzyme A thioesterase activity, choloyl-coenzyme A thioesterase activity Sources: EC:3.1.2.27